{
  "gene": "UniProtKB:Q96H78",
  "term_id": "GO:0005739",
  "term_label": "mitochondrion",
  "gene_name": "Solute carrier family 25 member 44",
  "gene_symbol": "SLC25A44"
}